{
  "gene": "UniProtKB:O15172",
  "gene_name": "Putative phosphoserine phosphatase-like protein",
  "term_id": "UNKNOWN:0003",
  "term_label": "Unknown cellular component",
  "gene_symbol": "PSPHP1"
}